N-malonyltransferase activity [GO:0050735] (molecular function) Sources: GOC:ai Relationships: is_a N-acyltransferase activity [GO:0016410]; is a type of malonyltransferase activity [GO:0016420] Definition: Catalysis of the transfer of a malonyl group to a nitrogen atom on the acceptor molecule. Subtypes: 3,4-dichloroaniline N-malonyltransferase activity [GO:0047163], anthranilate N-malonyltransferase activity [GO:0047673], D-tryptophan N-malonyltransferase activity [GO:0047836]